{
  "gene_symbol": "LPIN2",
  "gene": "UniProtKB:Q92539",
  "term_id": "GO:0005789",
  "gene_name": "Phosphatidate phosphatase LPIN2",
  "term_label": "endoplasmic reticulum membrane"
}